{
  "term_id": "UNKNOWN:0002",
  "gene": "UniProtKB:A8MZ25",
  "term_label": "Unknown biological process",
  "gene_name": "Putative uncharacterized protein FLJ38767",
  "gene_symbol": "A8MZ25"
}